nucleus-vacuole junction [GO:0071561] (cellular component) Also known as: NV junction, NVJ, nucleus-vacuole membrane contact site Definition: An organelle membrane contact site formed between the vacuole membrane and the outer nuclear membrane. In S. cerevisiae these contacts are mediated through direct physical interaction between Vac8p and Nvj1p. References: PMID:16709156, PMID:16806880 Sources: GOC:jp Relationships: is a type of GO:0044232